{
  "gene": "UniProtKB:A0A075B6W4",
  "term_id": "UNKNOWN:0002",
  "term_label": "Unknown biological process",
  "gene_name": "T cell receptor alpha joining 46 (Fragment)",
  "gene_symbol": "TRAJ46"
}